[heparan sulfate]-glucosamine 3-sulfotransferase activity [GO:0008467] (molecular function) Relationships: is a type of heparan sulfate sulfotransferase activity [GO:0034483] Definition: Catalysis of the reaction: alpha-D-glucosaminyl-[heparan sulfate](n) + 3'-phosphoadenylyl sulfate = 3-sulfo-alpha-D-glucosaminyl-[heparan sulfate](n) + adenosine 3',5'-bisphosphate + H+. Also known as: 3'-phosphoadenylyl-sulfate:[heparan sulfate]-glucosamine 3-sulfotransferase, [heparan sulfate]-glucosamine 3-sulfotransferase 1 activity, [heparan sulfate]-glucosamine 3-sulfotransferase 2 activity, [heparan sulfate]-glucosamine 3-sulfotransferase 3 activity, 3'-phosphoadenylyl-sulfate:heparin-glucosamine 3-O-sulfotransferase activity, 3-OST activity, glucosaminyl 3-O-sulfotransferase activity, heparan sulfate D-glucosaminyl 3-O-sulfotransferase activity, heparin-glucosamine 3-O-sulfotransferase activity, heparin-glucosamine 3-O-sulphotransferase activity Sources: RHEA:15461